{
  "gene": "UniProtKB:P05783",
  "gene_name": "Keratin, type I cytoskeletal 18",
  "gene_symbol": "KRT18",
  "term_id": "GO:0005856",
  "term_label": "cytoskeleton"
}